{
  "term_label": "transmembrane-ephrin receptor activity",
  "gene_name": "Ephrin type-B receptor 2",
  "gene_symbol": "EPHB2",
  "term_id": "GO:0005005",
  "gene": "UniProtKB:P29323"
}